{
  "gene_symbol": "MT1HL1",
  "gene": "UniProtKB:P0DM35",
  "term_id": "GO:0005737",
  "gene_name": "Metallothionein 1H-like protein 1",
  "term_label": "cytoplasm"
}